zymogen binding [GO:0035375] (MF) Sources: ISBN:0198506732 Relationships: is a type of enzyme binding [GO:0019899] Also known as: proenzyme binding Definition: Binding to a zymogen, an enzymatically inactive precursor of an enzyme that is often convertible to an active enzyme by proteolysis.